achromobactin biosynthetic process [GO:0042861] (BP) Relationships: is a type of GO:0019290; is a type of amide biosynthetic process [GO:0043604]; is a type of carboxylic acid biosynthetic process [GO:0046394] References: PMID:10928541 Sources: GOC:jl Definition: The chemical reactions and pathways resulting in the formation of achromobactin, a citrate siderophore. Also known as: achromobactin anabolism, achromobactin biosynthesis, achromobactin formation, achromobactin synthesis